thylakoid light-harvesting complex [GO:0009503] (cellular component) Definition: A thylakoid membrane complex of chlorophylls a and b together with chlorophyll a-b binding proteins. In addition, LHCs contain a number of other proteins, the function of which is speculative, together with accessory pigments. The LHCs capture and transfer energy to photosystems I and II. An example of this is found in Arabidopsis thaliana. Relationships: is a type of light-harvesting complex [GO:0030076]; is a type of chloroplast thylakoid membrane protein complex [GO:0098807] Subtypes: GO:0009517, PSI associated light-harvesting complex I [GO:0009518] Sources: GOC:mtg_sensu, ISBN:0198547684